terpene catabolic process [GO:0046247] (biological process) Subtypes: GO:0016121, isoprene catabolic process [GO:0043613], GO:0043694, sesquiterpene catabolic process [GO:0051763], ent-pimara-8(14),15-diene catabolic process [GO:1901540], miltiradiene catabolic process [GO:1901945] Sources: GOC:ai Definition: The chemical reactions and pathways resulting in the breakdown of terpenes, any of a large group of hydrocarbons made up of isoprene units. Relationships: is a type of isoprenoid catabolic process [GO:0008300]; is a type of GO:0042214; is a type of hydrocarbon catabolic process [GO:0120253] Also known as: terpene breakdown, terpene catabolism, terpene degradation